steroid receptor RNA activator RNA binding [GO:0002153] (MF) Note: Note: there is also evidence that the RNA itself may code a protein (solution structure of mouse steroid receptor RNA activator 1 (SRA1) protein submitted to PDB by Riken). Relationships: is a type of single-stranded RNA binding [GO:0003727] References: PMID:10199399, PMID:15180993 Sources: GOC:vw Definition: Binding to a steroid receptor RNA activator RNA (SRA). SRA enhances steroid hormone receptor transcriptional activity as an RNA transcript by an indirect mechanism that does not involve SRA-steroid receptor binding. Also known as: SRA binding